{
  "term_label": "phospholipid translocation",
  "gene_symbol": "ABCB1",
  "gene_name": "ATP-dependent translocase ABCB1",
  "term_id": "GO:0045332",
  "gene": "UniProtKB:P08183"
}